{
  "term_label": "Unknown cellular component",
  "gene": "UniProtKB:Q9UHW5",
  "gene_name": "GPN-loop GTPase 3",
  "term_id": "UNKNOWN:0003",
  "gene_symbol": "GPN3"
}